{
  "term_label": "Unknown cellular component",
  "gene_symbol": "FAAH2",
  "term_id": "UNKNOWN:0003",
  "gene": "UniProtKB:Q6GMR7",
  "gene_name": "Fatty-acid amide hydrolase 2"
}